{
  "term_label": "Unknown molecular function",
  "gene_name": "Zinc finger translocation-associated protein",
  "gene": "UniProtKB:C9JLR9",
  "term_id": "UNKNOWN:0001",
  "gene_symbol": "ZFTA"
}